sensory perception of temperature stimulus [GO:0050951] (biological process) Subtypes: thermoception [GO:0050955] Relationships: is a type of GO:0007600 Also known as: sensory perception of thermal stimulus Definition: The series of events required for an organism to receive a sensory temperature stimulus, convert it to a molecular signal, and recognize and characterize the signal. This is a neurological process. Sources: GOC:ai